{
  "gene_name": "PR domain zinc finger protein 14",
  "term_label": "regulation of transcription by RNA polymerase II",
  "term_id": "GO:0006357",
  "gene_symbol": "PRDM14",
  "gene": "UniProtKB:Q9GZV8"
}